inhibin complex binding [GO:0034710] (molecular function) Definition: Binding to an inhibin complex, a dimer of one inhibin-alpha subunit and one inhibin-beta subunit. Relationships: is a type of protein-containing complex binding [GO:0044877] Sources: GOC:BHF, GOC:mah